altruistic, chimeric, non-reproductive fruiting body development [GO:0099137] (biological process) References: PMID:18272966 Also known as: fully co-operative, chimeric, non-reproductive fruiting body development Relationships: is a type of chimeric non-reproductive fruiting body development [GO:0099136] Definition: Development of a chimeric, non-reproductive fruiting body in which cells of all genotypes have an equal chance of becoming a spore cell. Subtypes: altruistic, chimeric sorocarp development [GO:0099138]